{
  "term_id": "GO:0042285",
  "gene": "UniProtKB:Q8N3Y3",
  "term_label": "xylosyltransferase activity",
  "gene_symbol": "LARGE2",
  "gene_name": "Xylosyl- and glucuronyltransferase LARGE2"
}